protein transport along microtubule to mitotic spindle pole body [GO:1990976] (BP) Definition: The directed movement of a protein along a microtubule to the mitotic spindle pole body, mediated by motor proteins. References: PMID:25987607 Relationships: is a type of protein localization to mitotic spindle pole body [GO:1902440]; is a type of protein transport along microtubule to spindle pole body [GO:1990852]